regulation of toll-like receptor 21 signaling pathway [GO:2000443] (biological process) Relationships: is a type of regulation of toll-like receptor signaling pathway [GO:0034121]; regulates toll-like receptor 21 signaling pathway [GO:0035682] Also known as: regulation of TLR21 signaling pathway, regulation of toll-like receptor 21 signalling pathway Sources: GOC:obol Definition: Any process that modulates the frequency, rate or extent of toll-like receptor 21 signaling pathway. Subtypes: GO:2000444, GO:2000445